adenylylsulfate-ammonia adenylyltransferase activity [GO:0047352] (molecular function) Definition: Catalysis of the reaction: 5'-adenylyl sulfate + NH4 = adenosine 5'-phosphoramidate + 2 H+ + sulfate. Relationships: is a type of adenylyltransferase activity [GO:0070566] Also known as: adenylylsulphate-ammonia adenylyltransferase activity, APSAT, adenylylsulfate:ammonia adenylyltransferase activity Sources: EC:2.7.7.51, RHEA:19197